{
  "gene": "UniProtKB:Q9Y487",
  "term_label": "vacuolar proton-transporting V-type ATPase complex",
  "term_id": "GO:0016471",
  "gene_name": "V-type proton ATPase 116 kDa subunit a 2",
  "gene_symbol": "ATP6V0A2"
}